metanephric glomerulus vasculature development [GO:0072239] (biological process) Also known as: glomerulus capillary development Definition: The biological process whose specific outcome is the progression of a metanephric glomerulus vasculature from an initial condition to its mature state. This process begins with the formation of the metanephric glomerulus vasculature and ends with the mature structure. The metanephric glomerulus vasculature is composed of the tubule structures that carry blood or lymph in the metanephric glomerulus. Relationships: is a type of GO:0072012; is part of metanephric glomerulus development [GO:0072224] Sources: GOC:mtg_kidney_jan10